lactoperoxidase activity [GO:0140825] (molecular function) Relationships: is a type of peroxidase activity [GO:0004601] References: PMID:19339248 Sources: RHEA:56136 Definition: Catalysis of the reaction: 2 a phenolic donor + H2O2 = 2 a phenolic radical donor + 2 H2O. Also known as: peroxidase activity